{
  "gene_name": "Protein FAM223A",
  "term_label": "Unknown cellular component",
  "gene": "UniProtKB:Q8IWN6",
  "term_id": "UNKNOWN:0003",
  "gene_symbol": "FAM223A"
}